{
  "gene": "UniProtKB:Q96PM5",
  "term_id": "GO:0006511",
  "gene_name": "RING finger and CHY zinc finger domain-containing protein 1",
  "term_label": "ubiquitin-dependent protein catabolic process",
  "gene_symbol": "RCHY1"
}